{
  "gene": "UniProtKB:P00742",
  "term_id": "GO:0006508",
  "gene_symbol": "F10",
  "term_label": "proteolysis",
  "gene_name": "Coagulation factor X"
}